{
  "term_label": "protein unfolding",
  "gene": "UniProtKB:Q13608",
  "gene_symbol": "PEX6",
  "gene_name": "Peroxisomal ATPase PEX6",
  "term_id": "GO:0043335"
}